{
  "term_id": "GO:0016435",
  "gene_symbol": "MRM1",
  "gene": "UniProtKB:Q6IN84",
  "gene_name": "rRNA methyltransferase 1, mitochondrial",
  "term_label": "rRNA (guanine) methyltransferase activity"
}